positive regulation of ribosome biogenesis [GO:0090070] (biological process) Relationships: is a type of GO:0044089; is a type of regulation of ribosome biogenesis [GO:0090069]; positively regulates ribosome biogenesis [GO:0042254] Definition: Any process that increases the rate, frequency or extent of ribosome biogenesis. Ribosome biogenesis is the cellular process that results in the biosynthesis of constituent macromolecules, assembly, and arrangement of constituent parts of ribosome subunits. Sources: GOC:dph, GOC:tb